{
  "term_label": "Unknown molecular function",
  "gene": "UniProtKB:Q96A99",
  "term_id": "UNKNOWN:0001",
  "gene_symbol": "PTX4",
  "gene_name": "Pentraxin-4"
}